hypoglossal nerve morphogenesis [GO:0021618] (biological process) Definition: The process in which the anatomical structure of the hypoglossal nerve is generated and organized. This motor nerve innervates all the intrinsic and all but one of the extrinsic muscles of the tongue. Sources: GOC:cls, GOC:dgh, GOC:dph, GOC:jid, GO_REF:0000021 Also known as: CN XII morphogenesis Relationships: is_a GO:0021602; is part of hypoglossal nerve development [GO:0021566]